{
  "gene_symbol": "EFHC1",
  "term_label": "mitotic spindle organization",
  "gene_name": "EF-hand domain-containing protein 1",
  "gene": "UniProtKB:Q5JVL4",
  "term_id": "GO:0007052"
}